{
  "gene_name": "Regulator of microtubule dynamics protein 2",
  "gene_symbol": "RMDN2",
  "term_label": "microtubule binding",
  "term_id": "GO:0008017",
  "gene": "UniProtKB:Q96LZ7"
}